negative regulation of myotube differentiation [GO:0010832] (biological process) Definition: Any process that decreases the frequency, rate or extent of myotube differentiation. Myotube differentiation is the process in which a relatively unspecialized cell acquires specialized features of a myotube cell. Myotubes are multinucleated cells that are formed when proliferating myoblasts exit the cell cycle, differentiate and fuse. Relationships: is a type of GO:0010830; is a type of negative regulation of striated muscle cell differentiation [GO:0051154]; negatively regulates myotube differentiation [GO:0014902] Sources: GOC:dph, GOC:tb Subtypes: negative regulation of skeletal muscle fiber differentiation [GO:1902810]